S-linalool synthase activity [GO:0034007] (molecular function) Sources: EC:4.2.3.25, RHEA:24116 Also known as: 3S-linalool synthase activity, LIS, geranyl-diphosphate diphosphate-lyase [(3S)-linalool-forming] activity Relationships: is a type of carbon-oxygen lyase activity, acting on phosphates [GO:0016838] Definition: Catalysis of the reaction: geranyl diphosphate + H2O = (S)-linalool + diphosphate.